{
  "gene_symbol": "RAB8A",
  "term_label": "endosome",
  "gene_name": "Ras-related protein Rab-8A",
  "term_id": "GO:0005768",
  "gene": "UniProtKB:P61006"
}